{
  "gene_symbol": "DEFB119",
  "gene_name": "Beta-defensin 119",
  "gene": "UniProtKB:Q8N690",
  "term_label": "Unknown cellular component",
  "term_id": "UNKNOWN:0003"
}